{
  "gene": "UniProtKB:Q6XE24",
  "gene_name": "RNA-binding motif, single-stranded-interacting protein 3",
  "term_label": "Unknown biological process",
  "gene_symbol": "RBMS3",
  "term_id": "UNKNOWN:0002"
}